pteridine-containing compound metabolic process [GO:0042558] (biological process) Subtypes: folic acid-containing compound metabolic process [GO:0006760], pteridine metabolic process [GO:0019889], pteridine-containing compound biosynthetic process [GO:0042559], pteridine-containing compound catabolic process [GO:0042560], tetrahydrobiopterin metabolic process [GO:0046146], dihydrobiopterin metabolic process [GO:0051066], dihydropteridine metabolic process [GO:0051067], sarcinapterin metabolic process [GO:1900867], tatiopterin metabolic process [GO:1900869] Sources: GOC:jl, ISBN:0198506732 Definition: The chemical reactions and pathways involving any compound containing pteridine (pyrazino(2,3-dipyrimidine)), e.g. pteroic acid, xanthopterin and folic acid. Also known as: pteridine and derivative metabolic process, pteridine and derivative metabolism, pteridine-containing compound metabolism, pterin metabolic process, pterin metabolism Relationships: is a type of metabolic process [GO:0008152]